{
  "term_id": "GO:0016790",
  "term_label": "thiolester hydrolase activity",
  "gene_name": "Probable hydrolase PNKD",
  "gene": "UniProtKB:Q8N490",
  "gene_symbol": "PNKD"
}